positive regulation of oocyte maturation [GO:1900195] (biological process) Definition: Any process that activates or increases the frequency, rate or extent of oocyte maturation. Also known as: up regulation of oocyte maturation, up-regulation of oocyte maturation, upregulation of oocyte maturation, activation of oocyte maturation Relationships: is a type of regulation of oocyte maturation [GO:1900193]; is a type of GO:1903431; is a type of GO:2000243; positively regulates oocyte maturation [GO:0001556] Sources: GOC:TermGenie, GOC:kmv